neuronal cell body membrane [GO:0032809] (cellular component) Definition: The plasma membrane of a neuron cell body - excludes the plasma membrane of cell projections such as axons and dendrites. Sources: GOC:jl Also known as: neuron cell body membrane, neuronal cell soma membrane Relationships: is_a GO:0044298; is part of neuronal cell body [GO:0043025]